protein polyglycylation [GO:0018094] (biological process) Regulation: regulated by regulation of protein polyglycylation [GO:1903344]; negatively regulated by negative regulation of protein polyglycylation [GO:1903345]; positively regulated by positive regulation of protein polyglycylation [GO:1903346] Relationships: is_a peptidyl-glutamic acid modification [GO:0018200] Sources: RESID:AA0201 Definition: The addition of glycyl units covalently bound to the gamma carboxyl group peptidyl-glutamic acid.